{
  "gene": "UniProtKB:Q8N609",
  "gene_name": "Translocating chain-associated membrane protein 1-like 1",
  "term_label": "endoplasmic reticulum membrane",
  "term_id": "GO:0005789",
  "gene_symbol": "TRAM1L1"
}